{
  "term_label": "mitochondrion",
  "gene_name": "Parkinson disease protein 7",
  "gene_symbol": "PARK7",
  "term_id": "GO:0005739",
  "gene": "UniProtKB:Q99497"
}